DNA binding [GO:0003677] (molecular function) Subtypes: DNA secondary structure binding [GO:0000217], DNA template activity [GO:0000497], bent DNA binding [GO:0003681], damaged DNA binding [GO:0003684], double-stranded DNA binding [GO:0003690], GO:0003697, DNA binding, bending [GO:0008301], recombination hotspot binding [GO:0010844], chromatin DNA binding [GO:0031490], GO:0043565, DNA end binding [GO:0045027], triplex DNA binding [GO:0045142], GO:0051880, GO:0070336, GO:0099077 Sources: GOC:dph, GOC:jl, GOC:tb, GOC:vw Definition: Any molecular function by which a gene product interacts selectively and non-covalently with DNA (deoxyribonucleic acid). Regulation: positively regulated by GO:0043388; negatively regulated by GO:0043392; regulated by GO:0051101 Relationships: is a type of nucleic acid binding [GO:0003676] Also known as: plasmid binding, microtubule/chromatin interaction, structure specific DNA binding, structure-specific DNA binding